{
  "term_label": "Unknown biological process",
  "gene": "UniProtKB:Q9UBG7",
  "gene_symbol": "RBPJL",
  "term_id": "UNKNOWN:0002",
  "gene_name": "Recombining binding protein suppressor of hairless-like protein"
}